{
  "term_id": "UNKNOWN:0003",
  "term_label": "Unknown cellular component",
  "gene_symbol": "RNFT2",
  "gene_name": "RING finger and transmembrane domain-containing protein 2",
  "gene": "UniProtKB:Q96EX2"
}